{
  "gene_name": "Rho GTPase-activating protein 33",
  "gene_symbol": "ARHGAP33",
  "gene": "UniProtKB:O14559",
  "term_label": "postsynaptic density",
  "term_id": "GO:0014069"
}